epinephrine metabolic process [GO:0042414] (biological process) Definition: The chemical reactions and pathways involving epinephrine, a hormone produced by the medulla of the adrenal glands that increases heart activity, improves the power and prolongs the action of muscles, and increases the rate and depth of breathing. It is synthesized by the methylation of norepinephrine. Subtypes: epinephrine biosynthetic process [GO:0042418], GO:0042419 Sources: GOC:jl, ISBN:0192801023, ISBN:0198506732 Relationships: is a type of catecholamine metabolic process [GO:0006584] Also known as: adrenaline metabolic process, adrenaline metabolism, epinephrine metabolism